{
  "gene_name": "Charged multivesicular body protein 4a",
  "term_label": "late endosome to vacuole transport via multivesicular body sorting pathway",
  "gene_symbol": "CHMP4A",
  "term_id": "GO:0032511",
  "gene": "UniProtKB:Q9BY43"
}